venom-mediated increase of sensory perception of pain [GO:0044742] (biological process) Relationships: is a type of venom-mediated perturbation of nervous system process [GO:0140136] Also known as: allodynia, hyperalgesia References: PMID:23034652 Sources: GOC:fj, GOC:jl Definition: A process in which an organism initiates, promotes, or enhances sensory perception of pain in another organism via the action of a venom. Can manifest as allodynia, a condition that causes pain when a stimulus that normally wouldn't cause pain, or hyperalgesia, an increased sensitivity to feeling pain and an extreme response to pain.